fucose transmembrane transporter activity [GO:0015150] (molecular function) Definition: Enables the transfer of fucose from one side of a membrane to the other. Fucose is 6-deoxygalactose and has two enantiomers, D-fucose and L-fucose. Sources: GOC:ai, GOC:mtg_transport, ISBN:0815340729 Relationships: is a type of hexose transmembrane transporter activity [GO:0015149]; is part of fucose transmembrane transport [GO:0015756] Subtypes: fucose:proton symporter activity [GO:0015535]